{
  "gene_symbol": "PNO1",
  "term_id": "UNKNOWN:0002",
  "term_label": "Unknown biological process",
  "gene": "UniProtKB:Q9NRX1",
  "gene_name": "RNA-binding protein PNO1"
}